{
  "gene": "UniProtKB:Q14390",
  "term_id": "UNKNOWN:0003",
  "gene_name": "Glutathione hydrolase light chain 2",
  "gene_symbol": "GGTLC2",
  "term_label": "Unknown cellular component"
}